{
  "gene_name": "Myotubularin-related protein 8",
  "term_id": "GO:0106018",
  "gene_symbol": "MTMR8",
  "term_label": "phosphatidylinositol-3,5-bisphosphate phosphatase activity",
  "gene": "UniProtKB:Q96EF0"
}